inositol 1,4,5-trisphosphate receptor activity involved in regulation of postsynaptic cytosolic calcium levels [GO:0098695] (molecular function) Sources: GOC:dos Also known as: IP3 receptor activity involved in regulation of postsynaptic cytosolic calcium levels Relationships: is a type of inositol 1,4,5-trisphosphate-gated calcium channel activity [GO:0005220]; is part of regulation of postsynaptic cytosolic calcium ion concentration [GO:0099566] Definition: Any inositol 1,4,5-trisphosphate receptor activity that is involved in regulation of postsynaptic cytosolic calcium ion concentration.